{
  "gene_name": "Olfactory receptor 8B4",
  "term_label": "Unknown cellular component",
  "gene_symbol": "OR8B4",
  "term_id": "UNKNOWN:0003",
  "gene": "UniProtKB:Q96RC9"
}